{
  "term_id": "GO:0042734",
  "gene_symbol": "EFNB1",
  "term_label": "presynaptic membrane",
  "gene_name": "Ephrin-B1",
  "gene": "UniProtKB:P98172"
}